masculinization of hermaphroditic germ-line [GO:0042006] (biological process) Relationships: is a type of hermaphrodite germ-line sex determination [GO:0040021] Sources: GOC:ems Definition: The determination of male sex and sexual phenotype in the germ-line of the hermaphrodite. An example of this is found in Caenorhabditis elegans.